negative regulation of sister chromatid cohesion [GO:0045875] (biological process) Relationships: is a type of regulation of sister chromatid cohesion [GO:0007063]; is a type of negative regulation of cell cycle process [GO:0010948]; is a type of GO:2001251; negatively regulates GO:0007062 Subtypes: GO:0034092 Definition: Any process that stops, prevents, or reduces the frequency, rate or extent of sister chromatid cohesion. Also known as: down regulation of sister chromatid cohesion, down-regulation of sister chromatid cohesion, downregulation of sister chromatid cohesion, inhibition of sister chromatid cohesion Sources: GOC:go_curators